{
  "term_label": "brain development",
  "gene_symbol": "CDK5R2",
  "gene_name": "Cyclin-dependent kinase 5 activator 2",
  "term_id": "GO:0007420",
  "gene": "UniProtKB:Q13319"
}